{
  "term_label": "cytoplasm",
  "gene": "UniProtKB:Q9BT56",
  "term_id": "GO:0005737",
  "gene_name": "Spexin",
  "gene_symbol": "SPX"
}